silver ion transmembrane transport [GO:1902601] (biological process) Also known as: silver transmembrane transport Definition: The directed movement of silver (Ag+) ions across a membrane. Relationships: is a type of silver ion transport [GO:0015673]; is a type of monoatomic cation transmembrane transport [GO:0098655] Sources: GOC:TermGenie, GOC:pr, GO_REF:0000069